{
  "gene_symbol": "SGPP1",
  "gene": "UniProtKB:Q9BX95",
  "gene_name": "Sphingosine-1-phosphate phosphatase 1",
  "term_label": "endoplasmic reticulum membrane",
  "term_id": "GO:0005789"
}